{
  "term_label": "neuron projection",
  "gene_symbol": "FXR1",
  "gene": "UniProtKB:P51114",
  "gene_name": "RNA-binding protein FXR1",
  "term_id": "GO:0043005"
}